{
  "gene": "UniProtKB:P14209",
  "gene_name": "CD99 antigen",
  "term_label": "T cell extravasation",
  "gene_symbol": "CD99",
  "term_id": "GO:0072683"
}